{
  "gene_symbol": "TWF2",
  "term_id": "GO:0010591",
  "gene": "UniProtKB:Q6IBS0",
  "gene_name": "Twinfilin-2",
  "term_label": "regulation of lamellipodium assembly"
}